{
  "gene": "UniProtKB:O94818",
  "gene_symbol": "NOL4",
  "term_label": "Unknown molecular function",
  "term_id": "UNKNOWN:0001",
  "gene_name": "Nucleolar protein 4"
}